{
  "term_label": "endoplasmic reticulum unfolded protein response",
  "gene_symbol": "HERPUD1",
  "term_id": "GO:0030968",
  "gene": "UniProtKB:Q15011",
  "gene_name": "Homocysteine-responsive endoplasmic reticulum-resident ubiquitin-like domain member 1 protein"
}